{
  "term_label": "cytosol",
  "gene": "UniProtKB:P50851",
  "gene_symbol": "LRBA",
  "term_id": "GO:0005829",
  "gene_name": "Lipopolysaccharide-responsive and beige-like anchor protein"
}